{
  "term_id": "GO:0000978",
  "term_label": "RNA polymerase II cis-regulatory region sequence-specific DNA binding",
  "gene_symbol": "PLAG1",
  "gene": "UniProtKB:Q6DJT9",
  "gene_name": "Zinc finger protein PLAG1"
}